negative regulation of signal transduction by p53 class mediator [GO:1901797] (biological process) Also known as: down regulation of signal transduction by p53 class mediator, down-regulation of signal transduction by p53 class mediator, downregulation of signal transduction by p53 class mediator, inhibition of signal transduction by p53 class mediator Definition: Any process that stops, prevents or reduces the frequency, rate or extent of signal transduction by p53 class mediator. Sources: GOC:TermGenie Relationships: is a type of regulation of signal transduction by p53 class mediator [GO:1901796]; is a type of negative regulation of intracellular signal transduction [GO:1902532]; negatively regulates signal transduction by p53 class mediator [GO:0072331] Subtypes: GO:0043518, GO:1902254